{
  "gene_symbol": "BUB3",
  "gene": "UniProtKB:O43684",
  "term_id": "GO:1990298",
  "term_label": "bub1-bub3 complex",
  "gene_name": "Mitotic checkpoint protein BUB3"
}